negative regulation of interleukin-7 production [GO:0032716] (biological process) Relationships: is a type of negative regulation of cytokine production [GO:0001818]; is a type of regulation of interleukin-7 production [GO:0032676]; negatively regulates interleukin-7 production [GO:0032636] References: PMID:25962782 Sources: GOC:mah Definition: Any process that stops, prevents, or reduces the frequency, rate, or extent of interleukin-7 production. Also known as: down regulation of interleukin-7 production, down-regulation of interleukin-7 production, downregulation of interleukin-7 production, negative regulation of IL-7 production, inhibition of interleukin-7 production, negative regulation of interleukin-7 biosynthetic process, negative regulation of interleukin-7 secretion